pyruvate transmembrane transporter activity [GO:0050833] (MF) Also known as: monocarboxylate (lactate, pyruvate, mevalonate) uptake/efflux porter activity Sources: GOC:ai Relationships: is a type of monocarboxylic acid transmembrane transporter activity [GO:0008028]; is part of GO:1901475 Definition: Enables the transfer of pyruvate, 2-oxopropanoate, from one side of a membrane to the other. Subtypes: GO:0005477